NAD+ diphosphatase activity [GO:0000210] (molecular function) Sources: RHEA:11800 Also known as: NAD diphosphatase activity, NAD pyrophosphatase activity, NAD(+) pyrophosphatase activity, NAD+ phosphohydrolase activity, NAD+ pyrophosphatase activity, NADP pyrophosphatase activity, nicotinamide adenine dinucleotide pyrophosphatase activity Relationships: is a type of dinucleotide phosphatase activity [GO:0004551] Definition: Catalysis of the reaction: NAD+ + H2O = AMP + NMN.